rhombomere 8 structural organization [GO:0021676] (biological process) Also known as: rhombomere 8 structural organisation Sources: GOC:cls, GOC:dgh, GOC:dph, GOC:jid, GO_REF:0000021 Definition: The process that contributes to creating the structural organization of rhombomere 8. This process pertains to the physical shaping of a rudimentary structure. Rhombomeres are transverse segments of the developing rhombencephalon. Rhombomeres are lineage restricted, express different genes from one another, and adopt different developmental fates. Rhombomeres are numbered in an anterior to posterior order. Relationships: is a type of rhombomere structural organization [GO:0021595]; is part of rhombomere 8 morphogenesis [GO:0021674]